negative regulation of sporulation [GO:0043939] (biological process) Definition: Any process that stops, prevents, or reduces the frequency, rate or extent of sporulation, the process whose specific outcome is the progression of a spore over time, from its initiation to the mature structure. Subtypes: negative regulation of sporulation resulting in formation of a cellular spore [GO:0042174], negative regulation of conidium formation [GO:0075308], negative regulation of oomycete sporangium development [GO:0075324] Relationships: is a type of regulation of sporulation [GO:0043937]; is a type of GO:0051093; negatively regulates GO:0043934 Sources: GOC:pamgo_curators